{
  "term_label": "tRNA (cytidine-5-)-methyltransferase activity",
  "gene_symbol": "NSUN2",
  "term_id": "GO:0016428",
  "gene_name": "RNA cytosine C(5)-methyltransferase NSUN2",
  "gene": "UniProtKB:Q08J23"
}